{
  "gene_name": "Complement C2",
  "gene": "UniProtKB:P06681",
  "gene_symbol": "C2",
  "term_label": "Unknown cellular component",
  "term_id": "UNKNOWN:0003"
}